platelet morphogenesis [GO:0036344] (biological process) Definition: Generation and organization of a platelet, a non-nucleated disk-shaped cell formed by extrusion from megakaryocytes, found in the blood of all mammals, and mainly involved in blood coagulation. Sources: CL:0000233, GOC:BHF, GOC:vk Relationships: is a type of GO:0000902